RNA polymerase III hybrid type promoter sequence-specific DNA binding [GO:0001039] (MF) Also known as: RNA polymerase III hybrid type promoter DNA binding References: PMID:12381659 Sources: GOC:txnOH Definition: Binding to a sequence of DNA that is a part of a hybrid type promoter that controls transcription by RNA polymerase III (Pol III). A hybrid Pol III promoter contains both regulatory elements both upstream and downstream of the transcription initiation site. An example gene with such a promoter is the S. cerevisiae U6 gene. Relationships: is a type of RNA polymerase III cis-regulatory region sequence-specific DNA binding [GO:0000992]